{
  "gene_symbol": "TIGD3",
  "gene": "UniProtKB:Q6B0B8",
  "term_id": "GO:0005634",
  "gene_name": "Tigger transposable element-derived protein 3",
  "term_label": "nucleus"
}